{
  "gene_name": "Neurogenic locus notch homolog protein 3",
  "term_label": "cell surface",
  "gene": "UniProtKB:Q9UM47",
  "term_id": "GO:0009986",
  "gene_symbol": "NOTCH3"
}